venom-mediated perturbation of biological process [GO:0035738] (biological process) Relationships: is a type of modulation of process of another organism [GO:0035821] Definition: A process by which an organism alters or subverts a biological process in another organism via the action of a venom. Venoms are injected into the prey by a bite or a sting. Venoms cause their biological effects via the many toxins that they contain; some venoms are complex mixtures of toxins of differing types. Venoms can serve as predation mechanisms or defense responses. Also known as: envenomation, envenomation perturbing biological process, envenomation resulting in modification of morphology or physiology of other organism, envenomation resulting in modulation of process in another organism, envenomation resulting in modulation of process in other organism Subtypes: venom-mediated edema [GO:0044398], venom-mediated perturbation of mast cell degranulation [GO:0044479], venom-mediated perturbation of signal transduction [GO:0044509], venom-mediated perturbation of ion channel activity [GO:0044560], venom-mediated perturbation of blood circulation [GO:0140134], GO:0140136, venom-mediated perturbation of muscle system process [GO:0140137], venom-mediated suppression of blood coagulation, intrinsic pathway [GO:0140184] Sources: Wikipedia:Venom